{
  "gene_name": "Very-long-chain 3-oxoacyl-CoA reductase",
  "gene_symbol": "HSD17B12",
  "term_id": "GO:0005783",
  "gene": "UniProtKB:Q53GQ0",
  "term_label": "endoplasmic reticulum"
}